regulation of lymphatic vascular permeability [GO:1990185] (biological process) Relationships: is a type of GO:0043114; is a type of GO:1990183 References: PMID:23897233 Definition: Any process that modulates the extent to which lymphatic vessels can be pervaded by fluid.